{
  "gene_symbol": "CDRT15",
  "gene_name": "CMT1A duplicated region transcript 15 protein",
  "gene": "UniProtKB:Q96T59",
  "term_id": "UNKNOWN:0001",
  "term_label": "Unknown molecular function"
}